{
  "term_label": "Unknown molecular function",
  "gene_name": "V-type immunoglobulin domain-containing suppressor of T-cell activation",
  "gene": "UniProtKB:Q9H7M9",
  "gene_symbol": "VSIR",
  "term_id": "UNKNOWN:0001"
}